{
  "gene_symbol": "HAUS5",
  "gene": "UniProtKB:O94927",
  "term_id": "GO:0007098",
  "gene_name": "HAUS augmin-like complex subunit 5",
  "term_label": "centrosome cycle"
}